{
  "gene": "UniProtKB:P26447",
  "gene_symbol": "S100A4",
  "gene_name": "Protein S100-A4",
  "term_id": "GO:0005634",
  "term_label": "nucleus"
}